{
  "gene": "UniProtKB:Q9UL33",
  "term_label": "TRAPP complex",
  "term_id": "GO:0030008",
  "gene_symbol": "TRAPPC2L",
  "gene_name": "Trafficking protein particle complex subunit 2-like protein"
}